{
  "gene_name": "Immunoglobulin alpha Fc receptor",
  "term_label": "transmembrane signaling receptor activity",
  "gene": "UniProtKB:P24071",
  "gene_symbol": "FCAR",
  "term_id": "GO:0004888"
}